adhesion of symbiont hyphopodium to host [GO:0075070] (BP) Also known as: adhesion of symbiont hyphopodium to host during symbiotic interaction Relationships: is a type of GO:0075001 Definition: The attachment of a hyphopodium of the symbiont to its host via adhesion molecules. The host is defined as the larger of the organisms involved in a symbiotic interaction. Note: Note that this term should not be used to annotate gene products of the host. It should only be used to annotate those gene products from the symbiont involved in this process. Sources: GOC:pamgo_curators